{
  "gene": "UniProtKB:P17509",
  "gene_symbol": "HOXB6",
  "gene_name": "Homeobox protein Hox-B6",
  "term_label": "anterior/posterior pattern specification",
  "term_id": "GO:0009952"
}